{
  "gene": "UniProtKB:Q13936",
  "gene_symbol": "CACNA1C",
  "term_id": "GO:0098703",
  "term_label": "calcium ion import across plasma membrane",
  "gene_name": "Voltage-dependent L-type calcium channel subunit alpha-1C"
}